histone arginine deiminase activity [GO:0140794] (molecular function) Also known as: histone-arginine deiminase activity, histone citrullination Definition: Catalysis of the reaction: H2O + histone 3 L-arginyl = histone 3 L-citrullyl + NH4+, resulting in histone citrullination. Note: The substrate for histone deiminase may be methyl-arginine, rather than arginine (see PMID:35197210 and PMID:16567635). References: PMID:15339660 Subtypes: histone H4R3 arginine deiminase activity [GO:0140809], histone H1R54 arginine deiminase activity [GO:0140810], histone H2AR3 arginine deiminase activity [GO:0140811], GO:0141057 Relationships: is a type of protein-arginine deiminase activity [GO:0004668]; is a type of histone modifying activity [GO:0140993]